{
  "term_id": "GO:0005634",
  "gene": "UniProtKB:P23193",
  "term_label": "nucleus",
  "gene_name": "Transcription elongation factor A protein 1",
  "gene_symbol": "TCEA1"
}